{
  "gene_symbol": "THPO",
  "gene": "UniProtKB:P40225",
  "gene_name": "Thrombopoietin",
  "term_id": "GO:0070374",
  "term_label": "positive regulation of ERK1 and ERK2 cascade"
}